{
  "term_id": "GO:0086091",
  "gene_symbol": "SCN1B",
  "gene_name": "Sodium channel subunit beta-1",
  "term_label": "regulation of heart rate by cardiac conduction",
  "gene": "UniProtKB:Q07699"
}